{
  "gene": "UniProtKB:P59665",
  "gene_name": "Neutrophil defensin 1",
  "gene_symbol": "DEFA1B",
  "term_id": "GO:0050830",
  "term_label": "defense response to Gram-positive bacterium"
}